{
  "term_label": "2 iron, 2 sulfur cluster binding",
  "term_id": "GO:0051537",
  "gene_name": "Frataxin, mitochondrial",
  "gene": "UniProtKB:Q16595",
  "gene_symbol": "FXN"
}